{
  "gene_symbol": "SKOR1",
  "term_label": "negative regulation of BMP signaling pathway",
  "gene_name": "SKI family transcriptional corepressor 1",
  "gene": "UniProtKB:P84550",
  "term_id": "GO:0030514"
}